{
  "gene": "UniProtKB:Q902F9",
  "gene_name": "Endogenous retrovirus group K member 113 Env polyprotein",
  "term_id": "UNKNOWN:0003",
  "gene_symbol": "HERVK_113",
  "term_label": "Unknown cellular component"
}